{
  "gene_symbol": "SAMM50",
  "gene": "UniProtKB:Q9Y512",
  "gene_name": "Sorting and assembly machinery component 50 homolog",
  "term_label": "protein insertion into mitochondrial outer membrane",
  "term_id": "GO:0045040"
}